{
  "term_label": "photoreceptor outer segment",
  "gene_symbol": "OPN1MW2",
  "term_id": "GO:0001750",
  "gene_name": "Medium-wave-sensitive opsin 2",
  "gene": "UniProtKB:P0DN77"
}